interleukin-20-mediated signaling pathway [GO:0140866] (biological process) Also known as: IL-20-mediated signaling pathway, interleukin-20-mediated signalling pathway Definition: The series of molecular signals initiated by interleukin-20 binding to its receptor on the surface of a target cell, and ending with the regulation of a downstream cellular process, e.g. transcription. Relationships: is a type of cytokine-mediated signaling pathway [GO:0019221] References: PMID:34755534